galactitol catabolic process [GO:0019404] (biological process) Relationships: is a type of GO:0019402; is a type of hexitol catabolic process [GO:0019407] Sources: ISBN:0198506732 Also known as: galactitol breakdown, galactitol catabolism, galactitol degradation Definition: The chemical reactions and pathways resulting in the breakdown of galactitol, the hexitol derived by the reduction of the aldehyde group of either D- or L-galactose.